{
  "term_label": "Unknown molecular function",
  "term_id": "UNKNOWN:0001",
  "gene_symbol": "GNL2",
  "gene_name": "Nucleolar GTP-binding protein 2",
  "gene": "UniProtKB:Q13823"
}